dichloromuconate cycloisomerase activity [GO:0018852] (molecular function) Relationships: is a type of intramolecular lyase activity [GO:0016872] Definition: Catalysis of the reaction: 2,4-dichloro-2,5-dihydro-5-oxofuran-2-acetate = 2,4-dichloro-cis,cis-muconate. Sources: EC:5.5.1.11 Also known as: 2,4-dichloro-2,5-dihydro-5-oxofuran-2-acetate lyase (decyclizing)